{
  "gene_name": "Olfactory receptor 14A16",
  "term_id": "GO:0005549",
  "gene": "UniProtKB:Q8NHC5",
  "term_label": "odorant binding",
  "gene_symbol": "OR14A16"
}